establishment of viral latency [GO:0019043] (biological process) Sources: GOC:jl Subtypes: GO:0075713, establishment of episomal latency [GO:0075720] Definition: A process by which a virus establishes a latent state within its host, either as an integrated provirus within the host genome or as an episome, where viral genome remains in the cytoplasm or nucleus as distinct objects. Relationships: is a type of viral process [GO:0016032]; is part of viral latency [GO:0019042] Also known as: lysogenic commitment, phage lysogeny